{
  "term_id": "GO:0042273",
  "gene_name": "HEAT repeat-containing protein 3",
  "gene_symbol": "HEATR3",
  "term_label": "ribosomal large subunit biogenesis",
  "gene": "UniProtKB:Q7Z4Q2"
}